{
  "gene_symbol": "EEIG2",
  "gene": "UniProtKB:Q5T8I3",
  "term_id": "UNKNOWN:0001",
  "term_label": "Unknown molecular function",
  "gene_name": "EEIG family member 2"
}